{
  "gene_name": "RIMS-binding protein 3A",
  "gene_symbol": "RIMBP3",
  "term_id": "GO:0002177",
  "gene": "UniProtKB:Q9UFD9",
  "term_label": "manchette"
}